{
  "term_label": "monoatomic cation channel activity",
  "gene_symbol": "UNC80",
  "gene_name": "Protein unc-80 homolog",
  "gene": "UniProtKB:Q8N2C7",
  "term_id": "GO:0005261"
}